{
  "gene_symbol": "ZNF133",
  "term_id": "GO:0005634",
  "term_label": "nucleus",
  "gene": "UniProtKB:P52736",
  "gene_name": "Zinc finger protein 133"
}